{
  "gene_symbol": "LUZP1",
  "gene": "UniProtKB:Q86V48",
  "gene_name": "Leucine zipper protein 1",
  "term_id": "GO:0005813",
  "term_label": "centrosome"
}